positive regulation of receptor clustering [GO:1903911] (biological process) Also known as: up regulation of receptor clustering, up-regulation of receptor clustering, upregulation of receptor clustering, activation of receptor clustering Subtypes: positive regulation of skeletal muscle acetylcholine-gated channel clustering [GO:1904395], positive regulation of AMPA glutamate receptor clustering [GO:1904719] Relationships: is a type of GO:1903909; is a type of positive regulation of protein localization to membrane [GO:1905477]; positively regulates receptor clustering [GO:0043113] References: PMID:23575248 Sources: GOC:TermGenie, GOC:als, GO_REF:0000058 Definition: Any process that activates or increases the frequency, rate or extent of receptor clustering.